{
  "gene_name": "Mitoferrin-2",
  "term_label": "mitochondrial membrane",
  "gene_symbol": "SLC25A28",
  "gene": "UniProtKB:Q96A46",
  "term_id": "GO:0031966"
}